glucosylglycerol-phosphate synthase activity [GO:0033828] (molecular function) Also known as: ADP-glucose:sn-glycerol-3-phosphate 2-beta-D-glucosyltransferase activity, ADPglucose:sn-glycerol-3-phosphate 2-beta-D-glucosyltransferase activity, GG-phosphate synthase activity, GGPS, glucosyl-glycerol-phosphate synthase activity Relationships: is a type of GO:0046527 Definition: Catalysis of the reaction: sn-glycerol 3-phosphate + ADP-glucose = 2-O-(beta-D-glucosyl)-sn-glycerol 3-phosphate + ADP + H+. Sources: EC:2.4.1.213, RHEA:12881